{
  "term_id": "GO:0071880",
  "gene_name": "Alpha-1B adrenergic receptor",
  "gene": "UniProtKB:P35368",
  "gene_symbol": "ADRA1B",
  "term_label": "adenylate cyclase-activating adrenergic receptor signaling pathway"
}